beta-1,2,3,4,5,6-hexachlorocyclohexane metabolic process [GO:0018877] (biological process) Relationships: is a type of hexachlorocyclohexane metabolic process [GO:0019497] Also known as: beta-1,2,3,4,5,6-hexachlorocyclohexane metabolism Definition: The chemical reactions and pathways involving beta-1,2,3,4,5,6-hexachlorocyclohexane, a halogenated organic insecticide that has been used worldwide for agriculture and public health. Sources: UM-BBD_pathwayID:hch